{
  "gene_name": "Calmodulin-like protein 3",
  "gene": "UniProtKB:P27482",
  "term_id": "GO:0010880",
  "gene_symbol": "CALML3",
  "term_label": "regulation of release of sequestered calcium ion into cytosol by sarcoplasmic reticulum"
}